Gq/11-coupled serotonin receptor activity [GO:0001587] (molecular function) Definition: Combining with serotonin and transmitting the signal across the membrane by activation of the Gq/11 subunit of an associated cytoplasmic heterotrimeric G protein complex. The Gq/11 subunit subsequently activates phospholipase C and results in an increase in inositol triphosphate (IP3) levels. References: PMID:18571247, PMID:18703043 Sources: GOC:bf, GOC:mah Also known as: 5-HT2 receptor activity, serotonin receptor activity, coupled via Gq/11 Relationships: is a type of G protein-coupled serotonin receptor activity [GO:0004993]